{
  "gene_symbol": "PWWP2B",
  "term_id": "GO:0005654",
  "gene": "UniProtKB:Q6NUJ5",
  "gene_name": "PWWP domain-containing protein 2B",
  "term_label": "nucleoplasm"
}